RNA polymerase II-specific DNA-binding transcription factor binding [GO:0061629] (molecular function) Sources: GOC:dph, GOC:vw Definition: Binding to a sequence-specific DNA binding RNA polymerase II transcription factor, any of the factors that interact selectively and non-covalently with a specific DNA sequence in order to modulate transcription. Subtypes: nuclear receptor binding [GO:0016922], aryl hydrocarbon receptor binding [GO:0017162], Tat protein binding [GO:0030957], GO:0051059, GO:0051525, STAT family protein binding [GO:0097677] Also known as: RNA polymerase II sequence-specific DNA binding transcription factor binding, RNA polymerase II sequence-specific DNA-binding transcription factor binding, RNA polymerase II activating transcription factor binding, RNA polymerase II repressing transcription factor binding, RNA polymerase II transcription factor binding Relationships: is a type of DNA-binding transcription factor binding [GO:0140297]